{
  "term_label": "Unknown cellular component",
  "gene_symbol": "BRME1",
  "gene": "UniProtKB:Q0VDD7",
  "gene_name": "Break repair meiotic recombinase recruitment factor 1",
  "term_id": "UNKNOWN:0003"
}